{
  "term_label": "cell-cell adhesion mediated by cadherin",
  "term_id": "GO:0044331",
  "gene": "UniProtKB:Q9H159",
  "gene_name": "Cadherin-19",
  "gene_symbol": "CDH19"
}